astrocyte differentiation [GO:0048708] (biological process) References: PMID:15139015 Sources: GOC:vp Regulation: regulated by regulation of astrocyte differentiation [GO:0048710]; positively regulated by positive regulation of astrocyte differentiation [GO:0048711]; negatively regulated by negative regulation of astrocyte differentiation [GO:0048712] Definition: The process in which a relatively unspecialized cell acquires the specialized features of an astrocyte. An astrocyte is the most abundant type of glial cell. Astrocytes provide support for neurons and regulate the environment in which they function. Subtypes: forebrain astrocyte differentiation [GO:0021896], Bergmann glial cell differentiation [GO:0060020] Relationships: is a type of glial cell differentiation [GO:0010001]; is part of central nervous system development [GO:0007417]